chylomicron remnant clearance [GO:0034382] (biological process) Sources: GOC:BHF, GOC:mah, GOC:pde Definition: The process in which a chylomicron remnant is removed from the blood via receptor-mediated endocytosis into liver cells and its constituent parts degraded. Regulation: regulated by GO:0090320; positively regulated by positive regulation of chylomicron remnant clearance [GO:0090321] Relationships: is a type of GO:0071830